{
  "gene": "UniProtKB:P51654",
  "gene_symbol": "GPC3",
  "term_label": "plasma membrane",
  "gene_name": "Glypican-3",
  "term_id": "GO:0005886"
}